{
  "gene_name": "V-type proton ATPase subunit H",
  "term_label": "Unknown biological process",
  "gene_symbol": "ATP6V1H",
  "term_id": "UNKNOWN:0002",
  "gene": "UniProtKB:Q9UI12"
}